negative regulation of transcription initiation-coupled chromatin remodeling [GO:0160217] (biological process) Definition: Any process that stops, prevents or reduces the frequency, rate or extent of transcription initiation-coupled chromatin remodeling. References: PMID:33980486 Relationships: is a type of regulation of gene expression [GO:0010468]; is a type of negative regulation of chromatin organization [GO:1905268]; negatively regulates GO:0045815